fibroblast migration [GO:0010761] (biological process) Definition: Cell migration that is accomplished by extension and retraction of a fibroblast pseudopodium. A fibroblast is a connective tissue cell which secretes an extracellular matrix rich in collagen and other macromolecules. Sources: GOC:BHF, GOC:dph, GOC:tb Also known as: fibroblast cell migration Relationships: is a type of ameboidal-type cell migration [GO:0001667] Subtypes: hepatic stellate cell migration [GO:0061868] Regulation: RO_0002211 by regulation of fibroblast migration [GO:0010762]; positively regulated by positive regulation of fibroblast migration [GO:0010763]; negatively regulated by negative regulation of fibroblast migration [GO:0010764]